regulation of antigen processing and presentation of polysaccharide antigen via MHC class II [GO:0002601] (BP) Definition: Any process that modulates the frequency, rate, or extent of antigen processing and presentation of polysaccharide antigen via MHC class II. Relationships: is_a regulation of antigen processing and presentation of peptide or polysaccharide antigen via MHC class II [GO:0002580]; regulates GO:0002505 Subtypes: GO:0002602, GO:0002603 Also known as: regulation of polysaccharide antigen processing and presentation via MHC class II Sources: GOC:add